{
  "gene": "UniProtKB:Q9BZI1",
  "term_label": "nucleus",
  "gene_symbol": "IRX2",
  "term_id": "GO:0005634",
  "gene_name": "Iroquois-class homeodomain protein IRX-2"
}